{
  "gene": "UniProtKB:Q86T03",
  "gene_name": "Type 1 phosphatidylinositol 4,5-bisphosphate 4-phosphatase",
  "term_label": "phagocytic vesicle membrane",
  "term_id": "GO:0030670",
  "gene_symbol": "PIP4P1"
}